{
  "term_id": "GO:0003924",
  "gene": "UniProtKB:Q9NZQ0",
  "term_label": "GTPase activity",
  "gene_name": "DnaJ homolog subfamily C member 27",
  "gene_symbol": "DNAJC27"
}